{
  "gene_symbol": "ETFRF1",
  "gene_name": "Electron transfer flavoprotein regulatory factor 1",
  "term_label": "mitochondrion",
  "gene": "UniProtKB:Q6IPR1",
  "term_id": "GO:0005739"
}